{
  "gene_name": "Kielin_chordin-like protein",
  "term_label": "Unknown molecular function",
  "gene": "UniProtKB:Q6ZWJ8",
  "gene_symbol": "KCP",
  "term_id": "UNKNOWN:0001"
}